instar larval or pupal morphogenesis [GO:0048707] (biological process) Definition: The process, occurring during instar larval or pupal development, by which anatomical structures are generated and organized. Sources: GOC:mtg_sensu, GOC:rc Relationships: is a type of post-embryonic animal morphogenesis [GO:0009886]; is part of GO:0002165